{
  "term_id": "GO:0140431",
  "gene_name": "Abasic site processing protein HMCES",
  "term_label": "DNA-(abasic site) binding",
  "gene": "UniProtKB:Q96FZ2",
  "gene_symbol": "HMCES"
}